{
  "gene_symbol": "ZNF174",
  "term_label": "DNA-binding transcription factor activity, RNA polymerase II-specific",
  "gene": "UniProtKB:Q15697",
  "gene_name": "Zinc finger protein 174",
  "term_id": "GO:0000981"
}